{
  "gene_name": "Olfactory receptor 6N1",
  "term_id": "GO:0004984",
  "term_label": "olfactory receptor activity",
  "gene_symbol": "OR6N1",
  "gene": "UniProtKB:Q8NGY5"
}